{
  "gene_symbol": "CEP290",
  "gene_name": "Centrosomal protein of 290 kDa",
  "gene": "UniProtKB:O15078",
  "term_label": "kidney development",
  "term_id": "GO:0001822"
}